{
  "term_label": "cytosolic large ribosomal subunit",
  "term_id": "GO:0022625",
  "gene_symbol": "RPL32",
  "gene_name": "Large ribosomal subunit protein eL32",
  "gene": "UniProtKB:P62910"
}